{
  "term_id": "GO:0031012",
  "gene_name": "Spondin-2",
  "gene_symbol": "SPON2",
  "gene": "UniProtKB:Q9BUD6",
  "term_label": "extracellular matrix"
}